CCR7 chemokine receptor binding [GO:0031732] (molecular function) Sources: GOC:mah, GOC:nln Also known as: MIP-3 beta receptor binding, type 1 EBV-induced G-protein coupled receptor binding, CCR7 chemokine receptor ligand Definition: Binding to a CCR7 chemokine receptor. Relationships: is_a GO:0048020